{
  "gene_name": "Signal transducer and activator of transcription 5B",
  "gene_symbol": "STAT5B",
  "term_id": "GO:0005634",
  "term_label": "nucleus",
  "gene": "UniProtKB:P51692"
}